{
  "gene_name": "Transcription factor Jun",
  "gene": "UniProtKB:P05412",
  "term_label": "transcription regulator complex",
  "term_id": "GO:0005667",
  "gene_symbol": "JUN"
}